[acetyl-CoA carboxylase]-phosphatase activity [GO:0050406] (molecular function) Definition: Catalysis of the reaction: [acetyl-CoA carboxylase]-phosphate + H2O = [acetyl-CoA carboxylase] + phosphate. Sources: EC:3.1.3.44, MetaCyc:ACETYL-COA-CARBOXYLASE-PHOSPHATASE-RXN Relationships: is a type of phosphoprotein phosphatase activity [GO:0004721] Also known as: acetyl-CoA carboxylase-phosphatase activity, acetyl-CoA:carbon-dioxide ligase (ADP-forming)-phosphate phosphohydrolase activity